miRNA binding [GO:0035198] (molecular function) Definition: Binding to a microRNA, a 21-23 nucleotide RNA that is processed from a stem-loop RNA precursor (pre-miRNA) that is encoded within plant and animal genomes. Also known as: microRNA binding References: PMID:15066283 Relationships: is a type of regulatory RNA binding [GO:0061980] Subtypes: miRNA inhibitor activity via base-pairing [GO:0140869]